{
  "gene_symbol": "GSTT4",
  "term_id": "GO:0004364",
  "term_label": "glutathione transferase activity",
  "gene_name": "Glutathione S-transferase theta-4",
  "gene": "UniProtKB:A0A1W2PR19"
}